{
  "gene_name": "Moesin",
  "gene": "UniProtKB:P26038",
  "term_label": "apical part of cell",
  "term_id": "GO:0045177",
  "gene_symbol": "MSN"
}